fructan beta-(2,1)-fructosidase activity [GO:0033948] (molecular function) Definition: Catalysis of the hydrolysis of terminal, non-reducing (2->1) linked beta-D-fructofuranose residues in fructans. Relationships: is a type of hydrolase activity, hydrolyzing O-glycosyl compounds [GO:0004553] Sources: EC:3.2.1.153 Also known as: 1-FEH II, 1-FEH w1, 1-FEH w2, 1-fructan exohydrolase activity, beta-(2,1)-D-fructan fructohydrolase activity, beta-(2,1)-fructan exohydrolase activity, beta-(2,1)-linkage-specific fructan-beta-fructosidase activity